{
  "gene": "UniProtKB:Q8N4W9",
  "gene_name": "Zinc finger protein 808",
  "term_label": "nucleus",
  "term_id": "GO:0005634",
  "gene_symbol": "ZNF808"
}